deoxyribonucleoside diphosphate biosynthetic process [GO:0009189] (biological process) Sources: GOC:go_curators, ISBN:0198506732 Also known as: deoxyribonucleoside diphosphate anabolism, deoxyribonucleoside diphosphate biosynthesis, deoxyribonucleoside diphosphate formation, deoxyribonucleoside diphosphate synthesis Subtypes: purine deoxyribonucleoside diphosphate biosynthetic process [GO:0009183], GO:0009197 Definition: The chemical reactions and pathways resulting in the formation of a deoxyribonucleoside diphosphate, a compound consisting of a nucleobase linked to a deoxyribose sugar esterified with diphosphate on the sugar. Relationships: is a type of nucleoside diphosphate biosynthetic process [GO:0009133]